{
  "gene": "UniProtKB:Q13651",
  "gene_name": "Interleukin-10 receptor subunit alpha",
  "term_label": "plasma membrane",
  "term_id": "GO:0005886",
  "gene_symbol": "IL10RA"
}